{
  "gene_symbol": "ADAM29",
  "term_id": "GO:0005886",
  "term_label": "plasma membrane",
  "gene": "UniProtKB:Q9UKF5",
  "gene_name": "Disintegrin and metalloproteinase domain-containing protein 29"
}